{
  "gene_name": "Transcription factor Dp family member 3",
  "gene_symbol": "TFDP3",
  "term_id": "GO:0005634",
  "term_label": "nucleus",
  "gene": "UniProtKB:Q5H9I0"
}